{
  "term_label": "Unknown molecular function",
  "gene_name": "Pancreatic secretory granule membrane major glycoprotein GP2",
  "gene_symbol": "GP2",
  "gene": "UniProtKB:P55259",
  "term_id": "UNKNOWN:0001"
}